{
  "gene_symbol": "CABS1",
  "term_id": "GO:0005509",
  "term_label": "calcium ion binding",
  "gene_name": "Calcium-binding and spermatid-specific protein 1",
  "gene": "UniProtKB:Q96KC9"
}